{
  "gene": "UniProtKB:Q9UNW1",
  "term_id": "GO:0052745",
  "term_label": "inositol phosphate phosphatase activity",
  "gene_name": "Multiple inositol polyphosphate phosphatase 1",
  "gene_symbol": "MINPP1"
}